{
  "gene": "UniProtKB:P29377",
  "term_label": "calcium ion binding",
  "gene_symbol": "S100G",
  "gene_name": "Protein S100-G",
  "term_id": "GO:0005509"
}